{
  "gene": "UniProtKB:Q99525",
  "term_label": "nucleosome assembly",
  "term_id": "GO:0006334",
  "gene_name": "Histone H4-like protein type G",
  "gene_symbol": "H4C7"
}